{
  "gene_name": "Probable G-protein coupled receptor 149",
  "gene": "UniProtKB:Q86SP6",
  "term_id": "GO:0005886",
  "term_label": "plasma membrane",
  "gene_symbol": "GPR149"
}